{
  "gene_name": "Indoleamine 2,3-dioxygenase 1",
  "term_id": "GO:0005737",
  "gene_symbol": "IDO1",
  "gene": "UniProtKB:P14902",
  "term_label": "cytoplasm"
}